{
  "gene": "UniProtKB:Q7Z4S9",
  "gene_symbol": "SH2D6",
  "term_label": "cell surface receptor protein tyrosine kinase signaling pathway",
  "term_id": "GO:0007169",
  "gene_name": "SH2 domain-containing protein 6"
}